{
  "term_label": "exocytosis",
  "gene_symbol": "STX19",
  "term_id": "GO:0006887",
  "gene_name": "Syntaxin-19",
  "gene": "UniProtKB:Q8N4C7"
}